{
  "gene_name": "KRAB domain-containing protein (Fragment)",
  "term_label": "Unknown molecular function",
  "gene_symbol": "LOC344065",
  "gene": "UniProtKB:A0A087WZK3",
  "term_id": "UNKNOWN:0001"
}